phosphocholine phosphatase activity [GO:0052731] (molecular function) Definition: Catalysis of the reaction: phosphocholine + H2O = choline + phosphate. Sources: RHEA:10492 Also known as: 3X11A, PHOSPHO1, phosphoethanolamine phosphohydrolase activity Relationships: is a type of GO:0016791